{
  "gene": "UniProtKB:P31350",
  "gene_symbol": "RRM2",
  "term_id": "GO:0009263",
  "gene_name": "Ribonucleoside-diphosphate reductase subunit M2",
  "term_label": "deoxyribonucleotide biosynthetic process"
}